{
  "gene_symbol": "TFE3",
  "term_label": "regulation of transcription by RNA polymerase II",
  "term_id": "GO:0006357",
  "gene": "UniProtKB:P19532",
  "gene_name": "Transcription factor E3"
}